transcription antitermination factor activity, DNA binding [GO:0001073] (molecular function) Definition: Binds to DNA, typically within region of the promoter and transcribed region, to promote readthrough of a transcription termination site and thus extending the length of the RNA transcript produced. Examples of antitermination factors which bind DNA include the lambda Q protein. Relationships: is a type of transcription regulator activity [GO:0140110]; is part of transcription antitermination [GO:0031564] References: PMID:8332211 Sources: GOC:txnOH Also known as: DNA binding transcription antitermination factor activity